{
  "gene_symbol": "CDCA4",
  "gene_name": "Cell division cycle-associated protein 4",
  "term_id": "UNKNOWN:0002",
  "term_label": "Unknown biological process",
  "gene": "UniProtKB:Q9BXL8"
}